intermediate mesodermal cell fate specification [GO:0048398] (biological process) Also known as: intermediate mesoderm cell fate specification Regulation: regulated by regulation of intermediate mesodermal cell fate specification [GO:0048399]; positively regulated by positive regulation of intermediate mesodermal cell fate specification [GO:0048400]; negatively regulated by GO:0048401 Definition: The process in which a cell becomes capable of differentiating autonomously into an intermediate mesoderm cell in an environment that is neutral with respect to the developmental pathway; upon specification, the cell fate can be reversed. Sources: GOC:dgh Relationships: is a type of mesodermal cell fate specification [GO:0007501]; is part of GO:0048393